{
  "gene_symbol": "IFITM2",
  "gene": "UniProtKB:Q01629",
  "term_id": "GO:0035456",
  "gene_name": "Interferon-induced transmembrane protein 2",
  "term_label": "response to interferon-beta"
}